{
  "gene_symbol": "SCYL3",
  "gene_name": "Protein-associating with the carboxyl-terminal domain of ezrin",
  "term_id": "UNKNOWN:0001",
  "gene": "UniProtKB:Q8IZE3",
  "term_label": "Unknown molecular function"
}